{
  "term_label": "regulation of MAPK cascade",
  "gene_name": "GRB2-related adapter protein",
  "gene_symbol": "GRAP",
  "term_id": "GO:0043408",
  "gene": "UniProtKB:Q13588"
}